{
  "term_id": "GO:0098609",
  "gene_name": "V-set and immunoglobulin domain-containing protein 10-like 2",
  "term_label": "cell-cell adhesion",
  "gene": "UniProtKB:P0DP72",
  "gene_symbol": "VSIG10L2"
}